{
  "gene_name": "Phosphatidylinositol N-acetylglucosaminyltransferase subunit Q",
  "gene": "UniProtKB:Q9BRB3",
  "gene_symbol": "PIGQ",
  "term_label": "GPI anchor biosynthetic process",
  "term_id": "GO:0006506"
}